myosin filament [GO:0032982] (cellular component) Definition: A supramolecular fiber containing myosin heavy chains, plus associated light chains and other proteins, in which the myosin heavy chains are arranged into a filament. Also known as: myosin thick filament, thick filament Relationships: is a type of GO:0099512; has part myosin complex [GO:0016459] Subtypes: striated muscle myosin thick filament [GO:0005863], myosin II filament [GO:0097513] Sources: GOC:mah